primary amino compound catabolic process [GO:1901161] (biological process) Also known as: primary amino compound breakdown, primary amino compound catabolism, primary amino compound degradation Relationships: is a type of catabolic process [GO:0009056] Definition: The chemical reactions and pathways resulting in the breakdown of primary amino compound. Sources: GOC:TermGenie Subtypes: phenylethylamine catabolic process [GO:0019607], GO:0019635, serotonin catabolic process [GO:0042429], chrysobactin catabolic process [GO:0042859], GO:0046336